fascia adherens [GO:0005916] (cellular component) Definition: A cell-cell junction that contains the transmembrane protein N-cadherin, which interacts with identical molecules from neighbouring cells to form a tight mechanical intercellular link; forms a large portion of the intercalated disc, the structure at which myofibrils terminate in cardiomyocytes. References: PMID:11732910 Sources: GOC:aruk, GOC:bc, GOC:mtg_muscle Relationships: is_a cell-cell junction [GO:0005911]; is part of GO:0014704